{
  "gene_symbol": "MKI67",
  "gene_name": "Proliferation marker protein Ki-67",
  "term_id": "GO:0007088",
  "gene": "UniProtKB:P46013",
  "term_label": "regulation of mitotic nuclear division"
}